zinc ion import into lysosome [GO:0140916] (biological process) References: PMID:25808614 Definition: The directed import of zinc(2+) from the cytosol, across an organelle membrane, into a lysosome. Relationships: is a type of lysosomal transport [GO:0007041]; is a type of GO:0034486; is a type of zinc ion import into organelle [GO:0062111]